{
  "gene_symbol": "ECEL1",
  "term_id": "GO:0005886",
  "term_label": "plasma membrane",
  "gene": "UniProtKB:O95672",
  "gene_name": "Endothelin-converting enzyme-like 1"
}